L-fuconate dehydratase activity [GO:0050023] (MF) Definition: Catalysis of the reaction: L-fuconate = 2-dehydro-3-deoxy-L-fuconate + H2O. Sources: EC:4.2.1.68, RHEA:22772 Also known as: L-fuconate hydratase activity, L-fuconate hydro-lyase (2-dehydro-3-deoxy-L-fuconate-forming), L-fuconate hydro-lyase activity Relationships: is_a hydro-lyase activity [GO:0016836]